{
  "gene": "UniProtKB:E9PGG2",
  "term_id": "GO:0000978",
  "gene_symbol": "ANHX",
  "gene_name": "Anomalous homeobox protein",
  "term_label": "RNA polymerase II cis-regulatory region sequence-specific DNA binding"
}